{
  "gene_name": "Mitogen-activated protein kinase kinase kinase 20",
  "gene_symbol": "MAP3K20",
  "term_id": "GO:0007059",
  "term_label": "chromosome segregation",
  "gene": "UniProtKB:Q9NYL2"
}